dol-P-Man:Man(1)GlcN-acyl-PI alpha-1,6-mannosyltransferase activity [GO:0120563] (molecular function) Also known as: GPI-MT-II activity, glycosylphosphatidylinositol-mannosyltransferase II activity Definition: Catalysis of the transfer of an alpha-D-mannosyl residue from dolichol-P-mannose to Man(1)-GlcN-acyl-PI, forming an alpha-(1->6)-D-mannosyl-D-mannose linkage. This transfers the second mannose to the GPI precursor. Relationships: is a type of GO:0000009; is a type of GPI mannosyltransferase activity [GO:0004376] References: PMID:15623507